{
  "gene": "UniProtKB:P08887",
  "term_label": "interleukin-6-mediated signaling pathway",
  "term_id": "GO:0070102",
  "gene_symbol": "IL6R",
  "gene_name": "Interleukin-6 receptor subunit alpha"
}